cytoplasmic side of rough endoplasmic reticulum membrane [GO:0098556] (cellular component) Definition: The side (leaflet) of the rough endoplasmic reticulum membrane that faces the cytoplasm. Relationships: is a type of cytoplasmic side of endoplasmic reticulum membrane [GO:0098554]; BFO_0000050 rough endoplasmic reticulum membrane [GO:0030867] Sources: GOC:ab, GOC:dos